{
  "gene_name": "Putative protein N-methyltransferase FAM86B1",
  "gene_symbol": "FAM86B1",
  "gene": "UniProtKB:Q8N7N1",
  "term_id": "GO:0016279",
  "term_label": "protein-lysine N-methyltransferase activity"
}